{
  "gene": "UniProtKB:Q8WVE6",
  "term_id": "UNKNOWN:0001",
  "term_label": "Unknown molecular function",
  "gene_name": "Transmembrane protein 171",
  "gene_symbol": "TMEM171"
}